apoptotic body [GO:0097189] (CC) Definition: A vesicle containing parts of a dying cell. Apoptotic bodies can be formed during the execution phase of the apoptotic process, when the cell's cytoskeleton breaks up and causes the membrane to bulge outward. These bulges may separate from the cell, taking a portion of cytoplasm with them, to become apoptotic bodies. These are then engulfed by phagocytic cells, and their components recycled. Apoptotic bodies may range in size from 0.8 to 5um. References: PMID:15242875, PMID:24223256 Sources: GOC:mtg_apoptosis, GOC:vesicles, Wikipedia:Apoptosis, Wikipedia:Bleb_(cell_biology) Also known as: apoptotic vesicle, apoptotic bleb Relationships: is a type of extracellular vesicle [GO:1903561]